doxorubicin metabolic process [GO:0044598] (biological process) References: PMID:10200167 Relationships: is a type of GO:0016137; is a type of GO:0030638; is a type of primary alcohol metabolic process [GO:0034308]; is a type of ketone metabolic process [GO:0042180]; is a type of tertiary alcohol metabolic process [GO:1902644] Definition: The chemical reactions and pathways involving doxorubicin, an anthracycline antibiotic, used in cancer chemotherapy.